circadian regulation of calcium ion oscillation [GO:0010617] (biological process) Definition: Any process that modulates the concentration of cytosolic free calcium ion [Ca2+]cyt with a regularity of approximately 24 hours. Relationships: is a type of circadian rhythm [GO:0007623]; is a type of regulation of cytosolic calcium ion concentration [GO:0051480] Also known as: circadian regulation of cytosolic calcium ion homeostasis, circadian regulation of Ca2+ oscillation, circadian regulation of [Ca2+]cyt oscillation, circadian regulation of cytosolic free calcium ion oscillation References: PMID:17982000